{
  "gene_symbol": "VPS51",
  "gene": "UniProtKB:Q9UID3",
  "term_label": "Golgi organization",
  "term_id": "GO:0007030",
  "gene_name": "Vacuolar protein sorting-associated protein 51 homolog"
}